{
  "gene_name": "Heterogeneous nuclear ribonucleoprotein F",
  "gene": "UniProtKB:P52597",
  "term_label": "nucleoplasm",
  "term_id": "GO:0005654",
  "gene_symbol": "HNRNPF"
}